{
  "term_label": "carboxylic acid transmembrane transport",
  "gene": "UniProtKB:Q7RTY1",
  "gene_name": "Monocarboxylate transporter 9",
  "term_id": "GO:1905039",
  "gene_symbol": "SLC16A9"
}